multivesicular body membrane [GO:0032585] (cellular component) Also known as: MVB membrane, MVE membrane, multivesicular endosome membrane Relationships: is a type of late endosome membrane [GO:0031902]; is part of GO:0005771 Sources: GOC:mah Definition: The lipid bilayer surrounding a multivesicular body.